{
  "gene_name": "Follistatin",
  "gene_symbol": "FST",
  "term_label": "extracellular region",
  "gene": "UniProtKB:P19883",
  "term_id": "GO:0005576"
}